{
  "gene_name": "Sal-like protein 4",
  "term_id": "GO:0000981",
  "gene": "UniProtKB:Q9UJQ4",
  "gene_symbol": "SALL4",
  "term_label": "DNA-binding transcription factor activity, RNA polymerase II-specific"
}